{
  "term_id": "GO:0019901",
  "gene": "UniProtKB:Q92796",
  "term_label": "protein kinase binding",
  "gene_name": "Disks large homolog 3",
  "gene_symbol": "DLG3"
}